DNA replication termination region [GO:0097047] (cellular component) Definition: A chromosomal region that contains fork pausing elements influencing the progression and merging of DNA replication forks. Relationships: is a type of GO:0110165; is part of GO:0005694 Also known as: TER References: PMID:20797631 Sources: GOC:mcc, GOC:pr